T-helper 1 cell cytokine production [GO:0035744] (biological process) Relationships: is a type of CD4-positive, alpha-beta T cell cytokine production [GO:0035743]; is part of GO:0042088 Also known as: Th1 cell cytokine production Definition: Any process that contributes to cytokine production by a T-helper 1 cell. Note: Note that this term is in the subset of terms that should not be used for direct gene product annotation. Instead, select one of the 'regulation' children terms. Regulation: regulated by regulation of T-helper 1 cell cytokine production [GO:2000554]; negatively regulated by negative regulation of T-helper 1 cell cytokine production [GO:2000555]; positively regulated by GO:2000556 Sources: CL:0000545, GOC:BHF